transforming growth factor beta complex [GO:0099126] (cellular component) References: PMID:22943793 Sources: GOC:bhm Relationships: is a type of protein-containing complex [GO:0032991]; is part of extracellular matrix [GO:0031012] Also known as: TGF-beta complex, TGF-beta dimer, TGFB complex, TGFB dimer, TGFbeta complex, TGFbeta dimer Definition: A protein complex acting as ligand of the transforming growth factor beta receptor complex, typically a homodimer of any of the TFGbeta isoforms. The precursor of TGFbeta proteins is cleaved into mature TGFbeta and the latency-associated peptide (LAP), which remains non-covalently linked to mature TGFbeta rendering it inactive. TGFbeta is activated by dimerization and dissociation of the LAP.